{
  "gene": "UniProtKB:Q6ZR85",
  "term_id": "UNKNOWN:0003",
  "gene_name": "Uncharacterized protein C17orf107",
  "gene_symbol": "C17orf107",
  "term_label": "Unknown cellular component"
}